{
  "term_id": "GO:0006974",
  "gene_name": "Histone H2AX",
  "term_label": "DNA damage response",
  "gene_symbol": "H2AX",
  "gene": "UniProtKB:P16104"
}